{
  "gene_symbol": "DENND4A",
  "gene": "UniProtKB:Q7Z401",
  "term_id": "GO:0031410",
  "gene_name": "C-myc promoter-binding protein",
  "term_label": "cytoplasmic vesicle"
}